{
  "gene": "UniProtKB:Q8NCD3",
  "term_id": "GO:0034080",
  "gene_symbol": "HJURP",
  "gene_name": "Holliday junction recognition protein",
  "term_label": "CENP-A containing chromatin assembly"
}